{
  "gene_name": "Segment polarity protein dishevelled homolog DVL-2",
  "gene": "UniProtKB:O14641",
  "term_label": "cytosol",
  "term_id": "GO:0005829",
  "gene_symbol": "DVL2"
}